{
  "gene_symbol": "REV1",
  "term_label": "error-prone translesion synthesis",
  "gene": "UniProtKB:Q9UBZ9",
  "gene_name": "DNA repair protein REV1",
  "term_id": "GO:0042276"
}